{
  "gene": "UniProtKB:P51504",
  "term_id": "GO:0000981",
  "gene_name": "Zinc finger protein 80",
  "term_label": "DNA-binding transcription factor activity, RNA polymerase II-specific",
  "gene_symbol": "ZNF80"
}